{
  "term_label": "RNA polymerase II cis-regulatory region sequence-specific DNA binding",
  "term_id": "GO:0000978",
  "gene_symbol": "NPAS2",
  "gene": "UniProtKB:Q99743",
  "gene_name": "Neuronal PAS domain-containing protein 2"
}